leukocyte homeostasis [GO:0001776] (biological process) Note: Note that this term represents the return of immune system cell levels to stable numbers following an immune response as well as the proliferation and elimination of cells of the immune system required to maintain stable numbers in the absence of an outside stimulus. Subtypes: neutrophil homeostasis [GO:0001780], GO:0002260, mast cell homeostasis [GO:0033023], monocyte homeostasis [GO:0035702], dendritic cell homeostasis [GO:0036145], macrophage homeostasis [GO:0061519], eosinophil homeostasis [GO:1990959], basophil homeostasis [GO:1990960] Definition: The process of regulating the proliferation and elimination of cells of the immune system such that the total number of cells of a particular cell type within a whole or part of an organism is stable over time in the absence of an outside stimulus. Relationships: is a type of immune system process [GO:0002376]; is a type of homeostasis of number of cells [GO:0048872] Also known as: immune cell homeostasis, leucocyte homeostasis Sources: GOC:add, ISBN:0781735149